{
  "gene_name": "FMR1 neighbor protein",
  "term_id": "UNKNOWN:0002",
  "gene": "UniProtKB:Q8N0W7",
  "gene_symbol": "FMR1NB",
  "term_label": "Unknown biological process"
}